{
  "gene_symbol": "IGLL5",
  "term_label": "IgG immunoglobulin complex",
  "term_id": "GO:0071735",
  "gene_name": "Immunoglobulin lambda-like polypeptide 5",
  "gene": "UniProtKB:B9A064"
}